{
  "gene_name": "Protein piccolo",
  "term_id": "GO:0098978",
  "gene": "UniProtKB:Q9Y6V0",
  "term_label": "glutamatergic synapse",
  "gene_symbol": "PCLO"
}